{
  "term_label": "RNA binding",
  "term_id": "GO:0003723",
  "gene_symbol": "RPL37",
  "gene": "UniProtKB:P61927",
  "gene_name": "Large ribosomal subunit protein eL37"
}